MAP kinase tyrosine/serine/threonine phosphatase activity [GO:0017017] (molecular function) Definition: Catalysis of the reaction: MAP kinase serine/threonine/tyrosine phosphate + H2O = MAP kinase serine/threonine/tyrosine + phosphate. Also known as: dual-specificity MAP kinase phosphatase activity References: PMID:12184814 Sources: GOC:mah Relationships: is a type of protein tyrosine/serine/threonine phosphatase activity [GO:0008138]; is_a MAP kinase phosphatase activity [GO:0033549]